{
  "gene_symbol": "GATA5",
  "term_label": "nucleus",
  "term_id": "GO:0005634",
  "gene": "UniProtKB:Q9BWX5",
  "gene_name": "Transcription factor GATA-5"
}